isotype switching [GO:0045190] (biological process) Note: Note that IgM and IgD can be coexpressed by B cells via an alternate splicing mechanism, but true recombinational isotype switching to IgD has been demonstrated as well. Note that this term is best used to annotate gene products which are involved in the mechanism of DNA recombination used in isotype switching, like the B cell specific Swap70 factor in the mouse, rather than gene products which promote isotype switching such as cytokines or co-stimulatory molecules, which should instead be annotated to 'regulation of isotype switching ; GO:0045191'. Definition: The switching of activated B cells from IgM biosynthesis to biosynthesis of other isotypes of immunoglobulin, accomplished through a recombination process involving an intrachromosomal deletion involving switch regions that reside 5' of each constant region gene segment in the immunoglobulin heavy chain locus. Relationships: is a type of somatic recombination of immunoglobulin genes involved in immune response [GO:0002204]; is a type of B cell activation involved in immune response [GO:0002312] Regulation: regulated by GO:0045191; negatively regulated by negative regulation of isotype switching [GO:0045829]; positively regulated by positive regulation of isotype switching [GO:0045830] Subtypes: isotype switching to IgE isotypes [GO:0048289], isotype switching to IgA isotypes [GO:0048290], isotype switching to IgG isotypes [GO:0048291], isotype switching to IgD isotypes [GO:0048292] Sources: ISBN:0781735149 Also known as: class switch recombination, class switching, isotype switch recombination